{
  "term_id": "GO:0005737",
  "term_label": "cytoplasm",
  "gene_symbol": "ENSA",
  "gene_name": "Alpha-endosulfine",
  "gene": "UniProtKB:O43768"
}